callose deposition in phloem sieve plate [GO:0080165] (biological process) References: PMID:19470642 Definition: Any process in which callose is transported to, and/or maintained in, phloem sieve plate. Callose is a linear 1,3-beta-d-glucan formed from UDP-glucose and is found in certain plant cell walls. Relationships: is a type of callose localization [GO:0052545]